amyloplast starch grain [GO:0009568] (cellular component) Definition: Plant storage body for amylose and amylopectin, 1-100um in diameter, and located in amyloplasts. Also contains small amounts of enzymes, amino acids, lipids and nucleic acids. The shape of the grain varies widely amongst species, but is often spherical or disk-shaped. References: PMID:11217978 Sources: GOC:jl Also known as: amyloplast starch granule Relationships: is a type of GO:0043036; is part of amyloplast [GO:0009501]